{
  "gene_name": "Baculoviral IAP repeat-containing protein 8",
  "gene": "UniProtKB:Q96P09",
  "term_label": "nucleus",
  "term_id": "GO:0005634",
  "gene_symbol": "BIRC8"
}